{
  "term_label": "positive regulation of transcription by RNA polymerase II",
  "gene_name": "Phosphatidate phosphatase LPIN2",
  "term_id": "GO:0045944",
  "gene": "UniProtKB:Q92539",
  "gene_symbol": "LPIN2"
}